{
  "gene_symbol": "TM9SF2",
  "gene_name": "Transmembrane 9 superfamily member 2",
  "gene": "UniProtKB:Q99805",
  "term_label": "membrane",
  "term_id": "GO:0016020"
}